mRNA 5'-splice site recognition [GO:0000395] (biological process) Subtypes: alignment of 3' and 5' splice sites of mRNA [GO:0034403] Also known as: nuclear mRNA 5' splice site recognition, nuclear mRNA 5'-splice site recognition, U12-type nuclear mRNA 5' splice site recognition, U12-type nuclear mRNA 5'-splice site recognition, U2-type nuclear mRNA 5' splice site recognition, U2-type nuclear mRNA 5'-splice site recognition, spliceosomal CC complex biosynthesis, spliceosomal CC complex formation, spliceosomal E complex biosynthesis, spliceosomal E complex formation, spliceosomal commitment complex biosynthesis, spliceosomal commitment complex formation Relationships: is a type of mRNA splice site recognition [GO:0006376]; BFO_0000050 mRNA cis splicing, via spliceosome [GO:0045292] Note: Note that this step represents formation of the Commitment Complex (CC, in yeast) or the E complex (mammalian). Definition: Recognition of the intron 5'-splice site by components of the assembling spliceosome. Sources: GOC:krc, ISBN:0879695897